{
  "term_label": "cytoskeleton",
  "gene": "UniProtKB:Q9HCS5",
  "gene_symbol": "EPB41L4A",
  "gene_name": "Band 4.1-like protein 4A",
  "term_id": "GO:0005856"
}